{
  "term_label": "ATP-dependent chromatin remodeler activity",
  "term_id": "GO:0140658",
  "gene_symbol": "ERCC6",
  "gene_name": "DNA excision repair protein ERCC-6",
  "gene": "UniProtKB:Q03468"
}